{
  "gene": "UniProtKB:P17516",
  "term_id": "GO:0047023",
  "gene_name": "Aldo-keto reductase family 1 member C4",
  "gene_symbol": "AKR1C4",
  "term_label": "androsterone dehydrogenase [NAD(P)+] activity"
}